{
  "gene": "UniProtKB:P35240",
  "gene_symbol": "NF2",
  "term_label": "actin binding",
  "gene_name": "Merlin",
  "term_id": "GO:0003779"
}